{
  "term_label": "platelet-activating factor acetyltransferase activity",
  "gene": "UniProtKB:P68402",
  "gene_name": "Platelet-activating factor acetylhydrolase IB subunit alpha2",
  "gene_symbol": "PAFAH1B2",
  "term_id": "GO:0047179"
}